{
  "term_id": "GO:0005829",
  "gene": "UniProtKB:Q99707",
  "gene_name": "Methionine synthase",
  "term_label": "cytosol",
  "gene_symbol": "MTR"
}